{
  "gene_name": "CUB and sushi domain-containing protein 3",
  "term_id": "UNKNOWN:0001",
  "term_label": "Unknown molecular function",
  "gene": "UniProtKB:Q7Z407",
  "gene_symbol": "CSMD3"
}